positive regulation of response to nutrient levels [GO:0032109] (biological process) Sources: GOC:mah Also known as: up regulation of response to nutrient levels, up-regulation of response to nutrient levels, upregulation of response to nutrient levels, activation of response to nutrient levels, stimulation of response to nutrient levels Subtypes: positive regulation of sorocarp stalk cell differentiation [GO:0031287], positive regulation of response to food [GO:0032097], positive regulation of nitrogen utilization [GO:0045848], positive regulation of sulfur utilization [GO:0045883], positive regulation of cellular response to phosphate starvation [GO:0080040], GO:0110013, positive regulation of filamentous growth of a population of unicellular organisms in response to starvation [GO:1900436], positive regulation of cellular response to amino acid starvation [GO:1903833] Relationships: is a type of regulation of response to nutrient levels [GO:0032107]; is a type of positive regulation of response to stimulus [GO:0048584]; RO_0002213 response to nutrient levels [GO:0031667] Definition: Any process that activates or increases the frequency, rate or extent of a response to nutrient levels.